{
  "term_id": "GO:0004984",
  "gene": "UniProtKB:Q9Y585",
  "gene_symbol": "OR1A2",
  "term_label": "olfactory receptor activity",
  "gene_name": "Olfactory receptor 1A2"
}